{
  "term_label": "negative regulation of Notch signaling pathway",
  "gene_symbol": "DLL1",
  "gene_name": "Delta-like protein 1",
  "gene": "UniProtKB:O00548",
  "term_id": "GO:0045746"
}